{
  "gene_symbol": "TBC1D8B",
  "term_id": "GO:0005829",
  "term_label": "cytosol",
  "gene": "UniProtKB:Q0IIM8",
  "gene_name": "TBC1 domain family member 8B"
}